{
  "term_id": "GO:0071276",
  "term_label": "cellular response to cadmium ion",
  "gene": "UniProtKB:P80294",
  "gene_name": "Metallothionein-1H",
  "gene_symbol": "MT1H"
}